{
  "gene_symbol": "NAE1",
  "gene": "UniProtKB:Q13564",
  "gene_name": "NEDD8-activating enzyme E1 regulatory subunit",
  "term_label": "Unknown biological process",
  "term_id": "UNKNOWN:0002"
}